{
  "gene_symbol": "APOF",
  "gene": "UniProtKB:Q13790",
  "term_label": "cholesterol metabolic process",
  "gene_name": "Apolipoprotein F",
  "term_id": "GO:0008203"
}